regulation of actin filament-based movement [GO:1903115] (biological process) Subtypes: GO:0032971, regulation of hepatic stellate cell contraction [GO:0061873], regulation of cardiac muscle cell contraction [GO:0086004], regulation of apical constriction involved in ventral furrow formation [GO:0110073], positive regulation of actin filament-based movement [GO:1903116], regulation of myofibroblast contraction [GO:1904328] Relationships: is a type of regulation of actin filament-based process [GO:0032970]; regulates GO:0030048 References: PMID:24798735 Sources: GOC:TermGenie, GO_REF:0000058 Definition: Any process that modulates the frequency, rate or extent of actin filament-based movement.